{
  "gene_symbol": "CTSF",
  "term_label": "extracellular space",
  "gene_name": "Cathepsin F",
  "term_id": "GO:0005615",
  "gene": "UniProtKB:Q9UBX1"
}